methionine S-methyltransferase activity [GO:0030732] (MF) Definition: Catalysis of the reaction: S-adenosyl-L-methionine + L-methionine = S-adenosyl-L-homocysteine + S-methyl-L-methionine. Relationships: is a type of S-adenosylmethionine-dependent methyltransferase activity [GO:0008757] Also known as: S-adenosyl methionine:methionine methyl transferase activity, S-adenosyl-L-methionine:L-methionine S-methyltransferase activity, S-adenosylmethionine transmethylase activity, S-adenosylmethionine-methionine methyltransferase activity, methionine methyltransferase activity Sources: EC:2.1.1.12